regulation of thymocyte aggregation [GO:2000398] (BP) Subtypes: negative regulation of thymocyte aggregation [GO:2000399], GO:2000400 Sources: GOC:mah Definition: Any process that modulates the frequency, rate or extent of thymocyte aggregation. Also known as: regulation of T cell precursor aggregation, regulation of immature T-lymphocyte aggregation, regulation of thymic lymphocyte aggregation, regulation of immature T cell aggregation, regulation of immature T-cell aggregation Relationships: is a type of regulation of leukocyte cell-cell adhesion [GO:1903037]; regulates thymocyte aggregation [GO:0071594]